negative regulation of synaptic vesicle fusion to presynaptic active zone membrane [GO:0031631] (biological process) Relationships: is a type of negative regulation of vesicle fusion [GO:0031339]; is a type of regulation of synaptic vesicle fusion to presynaptic active zone membrane [GO:0031630]; is a type of negative regulation of synaptic vesicle membrane organization [GO:1901633]; is a type of GO:2000301; negatively regulates synaptic vesicle fusion to presynaptic active zone membrane [GO:0031629] Sources: GOC:mah Definition: Any process that stops, prevents, or reduces the frequency, rate or extent of synaptic vesicle fusion to the presynaptic membrane. Also known as: down regulation of synaptic vesicle fusion to presynaptic membrane, down-regulation of synaptic vesicle fusion to presynaptic membrane, downregulation of synaptic vesicle fusion to presynaptic membrane, inhibition of synaptic vesicle fusion to presynaptic membrane, negative regulation of synaptic vesicle fusion to pre-synaptic membrane, negative regulation of synaptic vesicle fusion to presynaptic membrane, down regulation of synaptic vesicle fusion to presynaptic active zone membrane, down-regulation of synaptic vesicle fusion to presynaptic active zone membrane, downregulation of synaptic vesicle fusion to presynaptic active zone membrane, negative regulation of synaptic vesicle fusion to pre-synaptic active zone membrane